{
  "gene_symbol": "CRNKL1",
  "gene": "UniProtKB:Q9BZJ0",
  "term_label": "U2-type catalytic step 2 spliceosome",
  "gene_name": "Crooked neck-like protein 1",
  "term_id": "GO:0071007"
}